adenine transmembrane transporter activity [GO:0015207] (molecular function) Relationships: is a type of purine nucleobase transmembrane transporter activity [GO:0005345]; is part of adenine transport [GO:0015853] Definition: Enables the transfer of adenine, 6-aminopurine, from one side of a membrane to the other. Sources: GOC:go_curators